{
  "gene_name": "TAR DNA-binding protein 43",
  "gene_symbol": "TARDBP",
  "term_label": "regulation of gene expression",
  "gene": "UniProtKB:Q13148",
  "term_id": "GO:0010468"
}